5-phosphoribose 1-diphosphate metabolic process [GO:0046391] (biological process) Relationships: is_a GO:0019693 Subtypes: 5-phosphoribose 1-diphosphate biosynthetic process [GO:0006015] Sources: GOC:ai Definition: The chemical reactions and pathways involving 5-phosphoribose 1-diphosphate, also known as 5-phosphoribosyl-1-pyrophosphate. Also known as: 5-phosphoribose 1-diphosphate metabolism, PRPP metabolic process